{
  "gene_symbol": "HYCC2",
  "gene_name": "Hyccin 2",
  "gene": "UniProtKB:Q8IXS8",
  "term_label": "plasma membrane",
  "term_id": "GO:0005886"
}